{
  "gene_symbol": "DCAF12",
  "term_id": "GO:0080008",
  "term_label": "Cul4-RING E3 ubiquitin ligase complex",
  "gene": "UniProtKB:Q5T6F0",
  "gene_name": "DDB1- and CUL4-associated factor 12"
}